serotonin secretion [GO:0001820] (biological process) Sources: GOC:ef, ISBN:0198506732, ISBN:0781735149 Subtypes: serotonin secretion involved in inflammatory response [GO:0002442], serotonin secretion, neurotransmission [GO:0060096] Relationships: is a type of GO:0006837; is a type of signal release [GO:0023061] Also known as: 5-HT secretion, 5-hydroxytryptamine secretion, serotonin release Definition: The regulated release of serotonin by a cell. Serotonin (5-hydroxytryptamine, or 5-HT) is a monoamine synthesized in serotonergic neurons in the central nervous system, enterochromaffin cells in the gastrointestinal tract and some immune system cells. Regulation: regulated by GO:0014062; negatively regulated by negative regulation of serotonin secretion [GO:0014063]; positively regulated by GO:0014064